{
  "gene": "UniProtKB:Q6NZY7",
  "gene_name": "Cdc42 effector protein 5",
  "term_id": "GO:0005886",
  "term_label": "plasma membrane",
  "gene_symbol": "CDC42EP5"
}